{
  "term_id": "GO:0030166",
  "term_label": "proteoglycan biosynthetic process",
  "gene_name": "Carbohydrate sulfotransferase 12",
  "gene_symbol": "CHST12",
  "gene": "UniProtKB:Q9NRB3"
}